7-cyano-7-deazaguanine metabolic process [GO:0097287] (biological process) Definition: The chemical reactions and pathways involving the Q nucleoside precursor 7-cyano-7-deazaguanine, also known as 2-amino-4-oxo-4,7-dihydro-3H-pyrrolo[2,3-d]pyrimidine-5-carbonitrile or preQo. References: PMID:364423 Sources: GOC:yaf Also known as: 7-cyano-7-deazaguanine metabolism Subtypes: GO:0097288 Relationships: is a type of GO:0050898